{
  "term_id": "GO:0001580",
  "gene_name": "Receptor-transporting protein 3",
  "gene_symbol": "RTP3",
  "gene": "UniProtKB:Q9BQQ7",
  "term_label": "detection of chemical stimulus involved in sensory perception of bitter taste"
}